{
  "term_id": "UNKNOWN:0002",
  "gene": "UniProtKB:Q96AT1",
  "gene_name": "Uncharacterized protein KIAA1143",
  "term_label": "Unknown biological process",
  "gene_symbol": "KIAA1143"
}